{
  "gene": "UniProtKB:Q08188",
  "gene_name": "Protein-glutamine gamma-glutamyltransferase E",
  "gene_symbol": "TGM3",
  "term_label": "keratinocyte differentiation",
  "term_id": "GO:0030216"
}